cystathionine gamma-lyase activity [GO:0004123] (molecular function) Definition: Catalysis of the reaction: L-cystathionine + H2O = 2-oxobutanoate + L-cysteine + NH4+. Sources: RHEA:14005 Relationships: is a type of carbon-sulfur lyase activity [GO:0016846] Also known as: L-cystathionine cysteine-lyase (deaminating), gamma-cystathionase activity, L-cystathionine cysteine-lyase (deaminating; 2-oxobutanoate-forming), homoserine deaminase activity, homoserine deaminase-cystathionase activity, homoserine dehydratase activity